nuclear estrogen receptor binding [GO:0030331] (molecular function) Definition: Binding to a nuclear estrogen receptor. Sources: GOC:ai Also known as: estrogen receptor binding Relationships: is a type of GO:0016922